{
  "gene_symbol": "ATF7",
  "term_label": "DNA-binding transcription factor activity, RNA polymerase II-specific",
  "gene": "UniProtKB:P17544",
  "gene_name": "Cyclic AMP-dependent transcription factor ATF-7",
  "term_id": "GO:0000981"
}